{
  "gene": "UniProtKB:Q7Z3V5",
  "gene_symbol": "ZNF571",
  "term_label": "nucleus",
  "gene_name": "Zinc finger protein 571",
  "term_id": "GO:0005634"
}